{
  "term_label": "RNA polymerase I core promoter sequence-specific DNA binding",
  "gene_symbol": "UBTFL1",
  "gene": "UniProtKB:P0CB47",
  "term_id": "GO:0001164",
  "gene_name": "Upstream-binding factor 1-like protein 1"
}